{
  "term_id": "GO:1905515",
  "gene_symbol": "FUZ",
  "gene_name": "Protein fuzzy homolog",
  "term_label": "non-motile cilium assembly",
  "gene": "UniProtKB:Q9BT04"
}